{
  "term_id": "GO:0042602",
  "gene": "UniProtKB:P30043",
  "gene_name": "Flavin reductase (NADPH)",
  "gene_symbol": "BLVRB",
  "term_label": "riboflavin reductase (NADPH) activity"
}